{
  "gene": "UniProtKB:Q8N6U8",
  "term_id": "GO:0007189",
  "gene_symbol": "GPR161",
  "term_label": "adenylate cyclase-activating G protein-coupled receptor signaling pathway",
  "gene_name": "G-protein coupled receptor 161"
}